anthocyanin 3'-O-beta-glucosyltransferase activity [GO:0033837] (molecular function) Relationships: is a type of GO:0046527 Also known as: 3'GT, UDP-glucose:anthocyanin 3'-O-beta-D-glucosyltransferase activity, UDP-glucose:anthocyanin 3'-O-glucosyltransferase activity Sources: EC:2.4.1.238 Definition: Catalysis of the reaction: UDP-glucose + an anthocyanin = UDP + an anthocyanin 3'-O-beta-D-glucoside.